silent mating-type cassette heterochromatin formation [GO:0030466] (biological process) Subtypes: GO:0140185 Also known as: chromatin silencing at silent mating-type cassette, heterochromatic silencing at silent mating-type cassette, silent mating type cassette region heterochromatin formation, silent mating-type cassette chromatin silencing, silent mating-type cassette heterochromatin assembly, silent-mating type cassette region heterochromatin formation, aging-dependent sterility, chromatin silencing at HML and HMR, establishment of chromatin silencing at silent mating-type cassette Relationships: is a type of constitutive heterochromatin formation [GO:0140719] Definition: Repression of transcription at silent mating-type loci by alteration of the structure of chromatin. Regulation: negatively regulated by negative regulation of silent mating-type cassette heterochromatin formation [GO:0061186]; regulated by regulation of silent mating-type cassette heterochromatin formation [GO:0090054]; positively regulated by positive regulation of silent mating-type cassette heterochromatin formation [GO:0090055] Sources: GOC:mcc